{
  "term_id": "GO:0005634",
  "gene_name": "E3 ubiquitin-protein ligase BRE1A",
  "term_label": "nucleus",
  "gene": "UniProtKB:Q5VTR2",
  "gene_symbol": "RNF20"
}